{
  "gene_symbol": "HNRNPUL2",
  "gene": "UniProtKB:Q1KMD3",
  "term_label": "alternative mRNA splicing, via spliceosome",
  "gene_name": "Heterogeneous nuclear ribonucleoprotein U-like protein 2",
  "term_id": "GO:0000380"
}